{
  "term_label": "positive regulation of acrosome reaction",
  "term_id": "GO:2000344",
  "gene_name": "Zona pellucida sperm-binding protein 3",
  "gene_symbol": "ZP3",
  "gene": "UniProtKB:P21754"
}